{
  "gene_name": "Sialin",
  "term_label": "sialic acid transport",
  "gene_symbol": "SLC17A5",
  "gene": "UniProtKB:Q9NRA2",
  "term_id": "GO:0015739"
}